{
  "gene_name": "E3 ubiquitin-protein ligase TRIM32",
  "gene": "UniProtKB:Q13049",
  "gene_symbol": "TRIM32",
  "term_id": "GO:0010508",
  "term_label": "positive regulation of autophagy"
}